{
  "gene": "UniProtKB:P51617",
  "gene_name": "Interleukin-1 receptor-associated kinase 1",
  "gene_symbol": "IRAK1",
  "term_label": "toll-like receptor 2 signaling pathway",
  "term_id": "GO:0034134"
}